{
  "gene": "UniProtKB:Q9H6H4",
  "gene_symbol": "REEP4",
  "gene_name": "Receptor expression-enhancing protein 4",
  "term_id": "GO:0071782",
  "term_label": "endoplasmic reticulum tubular network"
}